rRNA small subunit aminocarboxypropyltransferase activity [GO:0106388] (molecular function) References: PMID:27084949 Sources: RHEA:63296 Relationships: is a type of transferase activity, transferring alkyl or aryl (other than methyl) groups [GO:0016765]; is_a GO:0140102 Definition: Catalysis of the reaction: N1-methylpseudouridine in small subunit rRNA + S-adenosyl-L-methionine = H+ + N1-methyl-N3-[(3S)-3-amino-3-carboxypropyl]pseudouridine in small subunit rRNA + S-methyl-5'-thioadenosine. Also known as: 18S rRNA aminocarboxypropyltransferase activity